testosterone dehydrogenase (NAD+) activity [GO:0047035] (molecular function) Definition: Catalysis of the reaction: testosterone + NAD+ = androst-4-ene-3,17-dione + NADH. Relationships: is_a 17-beta-hydroxysteroid dehydrogenase (NAD+) activity [GO:0044594] Sources: RHEA:14929 Also known as: 17-beta-HSD activity, 17-ketoreductase activity, 3-alpha(17-beta)-hydroxysteroid dehydrogenase (NAD+) activity, 3alpha(17beta)-hydroxysteroid dehydrogenase (NAD+), 3alpha(or 17beta)-hydroxysteroid:NAD+ oxidoreductase activity, 3alpha,17beta-hydroxy steroid dehydrogenase activity, testosterone 17-beta-dehydrogenase (NAD+) activity, testosterone 17b-dehydrogenase activity, 17beta-HSD, 17beta-hydroxysteroid:NAD+ 17-oxidoreductase activity, 3alpha(17beta)-HSD, testosterone 17beta-dehydrogenase activity